{
  "gene": "UniProtKB:A0A1B0GUV7",
  "term_label": "Unknown molecular function",
  "gene_name": "Testis-expressed protein 48",
  "gene_symbol": "TEX48",
  "term_id": "UNKNOWN:0001"
}